{
  "term_label": "Unknown molecular function",
  "gene_name": "NEDD4-binding protein 3",
  "term_id": "UNKNOWN:0001",
  "gene_symbol": "N4BP3",
  "gene": "UniProtKB:O15049"
}